{
  "gene": "UniProtKB:O60663",
  "gene_symbol": "LMX1B",
  "term_label": "nucleus",
  "gene_name": "LIM homeobox transcription factor 1-beta",
  "term_id": "GO:0005634"
}